atf1-pcr1 complex [GO:1990243] (CC) Definition: A heterodimeric transcription factor complex composed of the bZIP proteins atf1 and pcr1. The heterodimer binds m26 sites (homologous to CRE). References: PMID:24224056 Relationships: is a type of transcription factor AP-1 complex [GO:0035976]